nerve growth factor binding [GO:0048406] (molecular function) Definition: Binding to nerve growth factor (NGF). Sources: GOC:dgh Also known as: NGF binding, beta-nerve growth factor binding, neurotrophin TRKA receptor activity Relationships: is a type of neurotrophin binding [GO:0043121]